3-chloro-D-alanine dehydrochlorinase activity [GO:0019149] (MF) Definition: Catalysis of the reaction: 3-chloro-D-alanine + H2O = pyruvate + chloride + NH3. Also known as: 3-chloro-D-alanine chloride-lyase (deaminating), 3-chloro-D-alanine chloride-lyase (deaminating; pyruvate-forming), beta-chloro-D-alanine dehydrochlorinase activity Relationships: is a type of carbon-halide lyase activity [GO:0016848] Sources: EC:4.5.1.2